{
  "gene_symbol": "EEF1AKMT2",
  "term_id": "GO:0016279",
  "term_label": "protein-lysine N-methyltransferase activity",
  "gene_name": "EEF1A lysine methyltransferase 2",
  "gene": "UniProtKB:Q5JPI9"
}